{
  "gene": "UniProtKB:O15218",
  "term_id": "UNKNOWN:0002",
  "term_label": "Unknown biological process",
  "gene_symbol": "GPR182",
  "gene_name": "G-protein coupled receptor 182"
}